{
  "term_label": "basement membrane",
  "gene_name": "Netrin-5",
  "term_id": "GO:0005604",
  "gene": "UniProtKB:Q8WTR8",
  "gene_symbol": "NTN5"
}